{
  "gene_symbol": "PCDHB6",
  "term_id": "GO:0007155",
  "gene_name": "Protocadherin beta-6",
  "term_label": "cell adhesion",
  "gene": "UniProtKB:Q9Y5E3"
}